T-helper 1 cell diapedesis [GO:0035688] (biological process) References: PMID:10477596 Sources: CL:0000545, GOC:BHF Also known as: Th1 cell diapedesis Definition: The passage of a T-helper 1 cell between the tight junctions of endothelial cells lining blood vessels, typically the fourth and final step of cellular extravasation. A T-helper 1 cell is a CD4-positive, alpha-beta T cell that has the phenotype T-bet-positive and produces interferon-gamma. Relationships: is a type of helper T cell diapedesis [GO:0035685]; is part of T-helper 1 cell extravasation [GO:0035687]